{
  "gene_symbol": "MALSU1",
  "term_label": "negative regulation of translation",
  "gene": "UniProtKB:Q96EH3",
  "term_id": "GO:0017148",
  "gene_name": "Mitochondrial assembly of ribosomal large subunit protein 1"
}